{
  "term_id": "GO:0030054",
  "gene_name": "Spectrin beta chain, non-erythrocytic 2",
  "gene_symbol": "SPTBN2",
  "gene": "UniProtKB:O15020",
  "term_label": "cell junction"
}